{
  "term_label": "L-proline transmembrane transporter activity",
  "gene": "UniProtKB:Q6YBV0",
  "term_id": "GO:0015193",
  "gene_name": "Neutral amino acid uniporter 4",
  "gene_symbol": "SLC36A4"
}